{
  "term_label": "regulation of immune system process",
  "gene_name": "Carcinoembryonic antigen-related cell adhesion molecule 20",
  "gene_symbol": "CEACAM20",
  "term_id": "GO:0002682",
  "gene": "UniProtKB:Q6UY09"
}